{
  "gene_name": "Sodium-dependent phosphate transport protein 1",
  "term_id": "GO:0015747",
  "gene_symbol": "SLC17A1",
  "term_label": "urate transport",
  "gene": "UniProtKB:Q14916"
}